{
  "gene_name": "4F2 cell-surface antigen heavy chain",
  "term_id": "GO:0016323",
  "gene": "UniProtKB:P08195",
  "gene_symbol": "SLC3A2",
  "term_label": "basolateral plasma membrane"
}